viral factory [GO:0039713] (cellular component) References: PMID:22440839 Sources: VZ:1951 Definition: An intracellular compartment in a host cell which increases the efficiency of viral replication, and shields the virus from host defenses. Viral factories can be either cytoplasmic or nuclear and often arise from extensive rearrangement of host cell cytoskeletal and/or cell membrane compartments. Also known as: virus factory Subtypes: cytoplasmic viral factory [GO:0039714], nuclear viral factory [GO:0039715] Relationships: is_a host cell part [GO:0033643]